bicyclomycin transmembrane transport [GO:0015905] (biological process) Definition: The directed movement of bicyclomycin across a lipid bilayer, from one side of a membrane to the other. Bicyclomycin (or bicozamycin) is an antibacterial drug often used as a livestock feed additive. References: PMID:20067529 Also known as: bicyclomycin transport Relationships: is a type of GO:0055085; is a type of GO:0071705